2-aminoethylphosphonate catabolic process [GO:0019635] (biological process) Sources: GOC:ai Relationships: is a type of phosphorus metabolic process [GO:0006793]; is a type of primary amino compound catabolic process [GO:1901161] Definition: The chemical reactions and pathways resulting in the breakdown of 2-aminoethylphosphonate, also known as ciliatine. Also known as: 2-aminoethylphosphonate breakdown, 2-aminoethylphosphonate catabolism, 2-aminoethylphosphonate degradation, 2-phosphonoethylamine catabolic process, 2-phosphonoethylamine catabolism, ciliatine catabolic process, ciliatine catabolism